lens fiber cell fate commitment [GO:0070308] (biological process) Relationships: is a type of cell fate commitment [GO:0045165]; is part of lens fiber cell differentiation [GO:0070306] Definition: The process in which the developmental fate of a cell becomes restricted such that it will develop into a lens fiber cell. A lens fiber cell is any of the elongated, tightly packed cells that make up the bulk of the mature lens in a camera-type eye. Also known as: lens fibre cell fate commitment References: PMID:7693735 Sources: GOC:mah